{
  "gene_symbol": "CHAC2",
  "term_id": "GO:0061928",
  "gene_name": "Glutathione-specific gamma-glutamylcyclotransferase 2",
  "term_label": "glutathione specific gamma-glutamylcyclotransferase activity",
  "gene": "UniProtKB:Q8WUX2"
}